lys-lys specific dibasic protein processing [GO:0090475] (biological process) Relationships: is a type of dibasic protein processing [GO:0090472] Definition: Any protein processing achieved by the cleavage of a peptide bond after two consecutive lysine amino acid residues within a protein. Sources: GOC:al